{
  "gene_name": "Butyrophilin subfamily 1 member A1",
  "gene_symbol": "BTN1A1",
  "gene": "UniProtKB:Q13410",
  "term_label": "regulation of cytokine production",
  "term_id": "GO:0001817"
}